long-chain fatty acid catabolic process [GO:0042758] (biological process) Note: While there is not universal consensus on the lengths of short-, medium-, long- and very-long-chain fatty acids, the GO uses the definitions in ChEBI (see CHEBI:26666, CHEBI:59554, CHEBI:15904 and CHEBI:27283). Relationships: is a type of long-chain fatty acid metabolic process [GO:0001676]; is_a GO:0009062 Also known as: long-chain fatty acid breakdown, long-chain fatty acid catabolism, long-chain fatty acid degradation References: PMID:20043225 Definition: The chemical reactions and pathways resulting in the breakdown of a long-chain fatty acid. A long-chain fatty acid has an aliphatic tail containing 13 to 22 carbons. Subtypes: leukotriene B4 catabolic process [GO:0036101], palmitic acid catabolic process [GO:1900534], GO:1901752